{
  "gene_name": "Nucleoside diphosphate kinase 3",
  "term_id": "GO:0004550",
  "gene_symbol": "NME3",
  "term_label": "nucleoside diphosphate kinase activity",
  "gene": "UniProtKB:Q13232"
}